{
  "term_label": "volume-sensitive chloride channel activity",
  "term_id": "GO:0072320",
  "gene": "UniProtKB:Q9H313",
  "gene_name": "Protein tweety homolog 1",
  "gene_symbol": "TTYH1"
}